syndecan-syntenin-ALIX complex [GO:1990562] (cellular component) References: PMID:22660413 Sources: GOC:bhm Relationships: is a type of extracellular exosome complex [GO:1990563] Also known as: exosome complex Definition: An exosome complex that is assembled in the multivesicular body (MVB) membrane and chaperoned to the exosome by the ESCRT-III machinery. Note: An example of this is SCD1 in human (UniProt symbol P18827) in PMID:22660413 (inferred from physical interaction).